{
  "term_id": "GO:0000086",
  "gene_name": "Tumor protein D53",
  "gene_symbol": "TPD52L1",
  "gene": "UniProtKB:Q16890",
  "term_label": "G2/M transition of mitotic cell cycle"
}